{
  "gene_name": "Nucleoporin Nup43",
  "term_label": "Unknown molecular function",
  "gene": "UniProtKB:Q8NFH3",
  "gene_symbol": "NUP43",
  "term_id": "UNKNOWN:0001"
}